{
  "gene_name": "Sulfhydryl oxidase 1",
  "gene_symbol": "QSOX1",
  "gene": "UniProtKB:O00391",
  "term_id": "GO:0005615",
  "term_label": "extracellular space"
}